{
  "gene": "UniProtKB:B4DX44",
  "gene_symbol": "ZNF736",
  "term_id": "GO:0000981",
  "term_label": "DNA-binding transcription factor activity, RNA polymerase II-specific",
  "gene_name": "Zinc finger protein 736"
}